{
  "term_label": "olfactory receptor activity",
  "gene": "UniProtKB:Q8NGL0",
  "gene_symbol": "OR5L2",
  "term_id": "GO:0004984",
  "gene_name": "Olfactory receptor 5L2"
}